{
  "gene_symbol": "KRT28",
  "gene_name": "Keratin, type I cytoskeletal 28",
  "gene": "UniProtKB:Q7Z3Y7",
  "term_label": "morphogenesis of an epithelium",
  "term_id": "GO:0002009"
}